{
  "gene_symbol": "WNT5B",
  "gene_name": "Protein Wnt-5b",
  "term_label": "cell fate commitment",
  "term_id": "GO:0045165",
  "gene": "UniProtKB:Q9H1J7"
}